{
  "gene": "UniProtKB:P33764",
  "gene_symbol": "S100A3",
  "term_id": "UNKNOWN:0002",
  "gene_name": "Protein S100-A3",
  "term_label": "Unknown biological process"
}